{
  "gene_symbol": "SEPTIN2",
  "term_id": "GO:0005940",
  "gene_name": "Septin-2",
  "gene": "UniProtKB:Q15019",
  "term_label": "septin ring"
}